{
  "gene_name": "Putative metallothionein MT1DP",
  "term_id": "GO:0046872",
  "gene": "UniProtKB:A1L3X4",
  "gene_symbol": "MT1DP",
  "term_label": "metal ion binding"
}